{
  "gene_symbol": "TP53",
  "term_label": "positive regulation of transcription by RNA polymerase II",
  "term_id": "GO:0045944",
  "gene_name": "Cellular tumor antigen p53",
  "gene": "UniProtKB:P04637"
}